{
  "gene_name": "Collagen alpha-1(XXII) chain",
  "term_label": "extracellular matrix structural constituent conferring tensile strength",
  "term_id": "GO:0030020",
  "gene_symbol": "COL22A1",
  "gene": "UniProtKB:Q8NFW1"
}